{
  "gene_symbol": "METTL6",
  "term_label": "Unknown molecular function",
  "term_id": "UNKNOWN:0001",
  "gene_name": "tRNA N(3)-methylcytidine methyltransferase METTL6",
  "gene": "UniProtKB:Q8TCB7"
}